{
  "term_label": "RNA binding",
  "gene_symbol": "DHX37",
  "term_id": "GO:0003723",
  "gene": "UniProtKB:Q8IY37",
  "gene_name": "Probable ATP-dependent RNA helicase DHX37"
}